{
  "term_id": "GO:0005634",
  "term_label": "nucleus",
  "gene_symbol": "EVX1",
  "gene_name": "Homeobox even-skipped homolog protein 1",
  "gene": "UniProtKB:P49640"
}